positive regulation of phosphatidylserine biosynthetic process [GO:1900470] (biological process) References: PMID:8056324, PMID:8614637 Sources: GOC:TermGenie, GOC:dgf Also known as: activation of phosphatidylserine anabolism, activation of phosphatidylserine biosynthesis, activation of phosphatidylserine formation, activation of phosphatidylserine synthesis, positive regulation of phosphatidylserine anabolism, positive regulation of phosphatidylserine biosynthesis, positive regulation of phosphatidylserine formation, positive regulation of phosphatidylserine synthesis, up regulation of phosphatidylserine anabolism, up regulation of phosphatidylserine biosynthesis, up regulation of phosphatidylserine biosynthetic process, up regulation of phosphatidylserine formation, up regulation of phosphatidylserine synthesis, up-regulation of phosphatidylserine anabolism, up-regulation of phosphatidylserine biosynthesis, up-regulation of phosphatidylserine biosynthetic process, up-regulation of phosphatidylserine formation, up-regulation of phosphatidylserine synthesis, upregulation of phosphatidylserine anabolism, upregulation of phosphatidylserine biosynthesis, upregulation of phosphatidylserine biosynthetic process, upregulation of phosphatidylserine formation, upregulation of phosphatidylserine synthesis, activation of phosphatidylserine biosynthetic process Relationships: is a type of positive regulation of phospholipid biosynthetic process [GO:0071073]; is a type of regulation of phosphatidylserine biosynthetic process [GO:1900468]; positively regulates phosphatidylserine biosynthetic process [GO:0006659] Definition: Any process that activates or increases the frequency, rate or extent of phosphatidylserine biosynthetic process.